{
  "term_label": "L-alanine transport",
  "gene_name": "Proton-coupled amino acid transporter 3",
  "gene": "UniProtKB:Q495N2",
  "gene_symbol": "SLC36A3",
  "term_id": "GO:0015808"
}